{
  "gene": "UniProtKB:Q06945",
  "term_label": "nucleus",
  "term_id": "GO:0005634",
  "gene_name": "Transcription factor SOX-4",
  "gene_symbol": "SOX4"
}